{
  "gene_name": "Mediator of RNA polymerase II transcription subunit 27",
  "term_label": "transcription coactivator activity",
  "term_id": "GO:0003713",
  "gene_symbol": "MED27",
  "gene": "UniProtKB:Q6P2C8"
}